{
  "term_label": "cell adhesion",
  "gene_name": "Cadherin-related family member 4",
  "term_id": "GO:0007155",
  "gene_symbol": "CDHR4",
  "gene": "UniProtKB:A6H8M9"
}